{
  "gene": "UniProtKB:O00445",
  "term_id": "GO:0005886",
  "gene_name": "Synaptotagmin-5",
  "gene_symbol": "SYT5",
  "term_label": "plasma membrane"
}